{
  "gene_name": "DNA-directed RNA polymerase II subunit GRINL1A",
  "gene_symbol": "POLR2M",
  "gene": "UniProtKB:P0CAP2",
  "term_id": "GO:0051685",
  "term_label": "maintenance of ER location"
}